{
  "term_label": "Unknown cellular component",
  "gene_symbol": "SREK1IP1",
  "term_id": "UNKNOWN:0003",
  "gene_name": "Protein SREK1IP1",
  "gene": "UniProtKB:Q8N9Q2"
}